isoamylase complex [GO:0043033] (cellular component) Also known as: debranching enzyme complex References: PMID:10333591 Sources: GOC:jl Definition: A protein complex whose composition varies amongst species; in rice it probably exists in a homo-tetramer to homo-hexamer form and in Gram-negative bacteria as a dimer. Functions in the hydrolysis of alpha-(1,6)-D-glucosidic branch linkages. Subtypes: GO:0010367, chloroplast isoamylase complex [GO:0010368] Relationships: is a type of catalytic complex [GO:1902494]